{
  "term_label": "Unknown molecular function",
  "gene_name": "Transmembrane protein 234",
  "gene_symbol": "TMEM234",
  "gene": "UniProtKB:Q8WY98",
  "term_id": "UNKNOWN:0001"
}